{
  "gene": "UniProtKB:O43508",
  "term_id": "GO:0006955",
  "term_label": "immune response",
  "gene_name": "Tumor necrosis factor ligand superfamily member 12",
  "gene_symbol": "TNFSF12"
}